{
  "gene_symbol": "CR1",
  "term_label": "extracellular space",
  "gene": "UniProtKB:P17927",
  "gene_name": "Complement receptor type 1",
  "term_id": "GO:0005615"
}